{
  "term_id": "GO:0098609",
  "gene_name": "Integrin alpha-11",
  "gene": "UniProtKB:Q9UKX5",
  "term_label": "cell-cell adhesion",
  "gene_symbol": "ITGA11"
}